{
  "gene_symbol": "RGL2",
  "gene_name": "Ral guanine nucleotide dissociation stimulator-like 2",
  "term_label": "Unknown molecular function",
  "gene": "UniProtKB:O15211",
  "term_id": "UNKNOWN:0001"
}